{
  "term_label": "protein kinase C binding",
  "gene": "UniProtKB:Q969G5",
  "gene_name": "Caveolae-associated protein 3",
  "gene_symbol": "CAVIN3",
  "term_id": "GO:0005080"
}